{
  "term_label": "Unknown biological process",
  "gene_name": "Coiled-coil domain-containing protein 146",
  "term_id": "UNKNOWN:0002",
  "gene_symbol": "CCDC146",
  "gene": "UniProtKB:Q8IYE0"
}